{
  "term_id": "UNKNOWN:0003",
  "term_label": "Unknown cellular component",
  "gene": "UniProtKB:Q86W10",
  "gene_name": "Cytochrome P450 4Z1",
  "gene_symbol": "CYP4Z1"
}